{
  "term_id": "UNKNOWN:0001",
  "gene_symbol": "KRTAP20-4",
  "gene": "UniProtKB:Q3LI62",
  "term_label": "Unknown molecular function",
  "gene_name": "Putative keratin-associated protein 20-4"
}